{
  "gene_symbol": "OVCA2",
  "term_label": "hydrolase activity",
  "gene": "UniProtKB:Q8WZ82",
  "term_id": "GO:0016787",
  "gene_name": "Esterase OVCA2"
}